{
  "gene_name": "Uncharacterized protein C20orf203",
  "gene_symbol": "C20orf203",
  "gene": "UniProtKB:Q8NBC4",
  "term_label": "Unknown molecular function",
  "term_id": "UNKNOWN:0001"
}